'de novo' UMP biosynthetic process [GO:0044205] (biological process) Sources: GOC:ecd, GOC:jl Also known as: 'de novo' UMP biosynthesis Definition: The chemical reactions and pathways resulting in the formation of UMP, uridine monophosphate, starting with the synthesis of (S)-dihydroorotate from bicarbonate; UMP biosynthesis may either occur via reduction by quinone, NAD+ or oxygen. Relationships: is a type of UMP biosynthetic process [GO:0006222]